{
  "gene_name": "Autophagy-related protein 2 homolog A",
  "gene_symbol": "ATG2A",
  "gene": "UniProtKB:Q2TAZ0",
  "term_id": "GO:0061908",
  "term_label": "phagophore"
}